interleukin-16 production [GO:0032619] (biological process) Relationships: is a type of cytokine production [GO:0001816] Definition: The appearance of interleukin-16 due to biosynthesis or secretion following a cellular stimulus, resulting in an increase in its intracellular or extracellular levels. Also known as: IL-16 production, pro-interleukin-16 production, LCF production, interleukin-16 biosynthetic process, interleukin-16 secretion Regulation: regulated by GO:0032659; negatively regulated by negative regulation of interleukin-16 production [GO:0032699]; positively regulated by positive regulation of interleukin-16 production [GO:0032739] Sources: GOC:mah